hydrogen peroxide transmembrane transport [GO:0080170] (biological process) Sources: GOC:tb Note: Note that this term is not intended for use in annotating lateral movement within membranes. Relationships: is a type of transmembrane transport [GO:0055085] Definition: The process in which hydrogen peroxide is transported across a membrane. Also known as: hydrogen peroxide membrane transport